{
  "term_label": "Unknown molecular function",
  "term_id": "UNKNOWN:0001",
  "gene": "UniProtKB:Q8TEM1",
  "gene_name": "Nuclear pore membrane glycoprotein 210",
  "gene_symbol": "NUP210"
}